{
  "gene_symbol": "RAP1GAP",
  "term_id": "GO:0005096",
  "term_label": "GTPase activator activity",
  "gene": "UniProtKB:P47736",
  "gene_name": "Rap1 GTPase-activating protein 1"
}